{
  "gene_name": "Immunoglobulin heavy constant mu",
  "term_label": "Unknown biological process",
  "gene": "UniProtKB:P01871",
  "gene_symbol": "IGHM",
  "term_id": "UNKNOWN:0002"
}